{
  "gene_name": "Nuclear pore complex-interacting protein family member B8",
  "gene_symbol": "NPIPB8",
  "term_id": "UNKNOWN:0003",
  "term_label": "Unknown cellular component",
  "gene": "UniProtKB:E9PQR5"
}